{
  "gene_symbol": "KRTAP20-3",
  "term_id": "UNKNOWN:0002",
  "term_label": "Unknown biological process",
  "gene_name": "Keratin-associated protein 20-3",
  "gene": "UniProtKB:Q3LI60"
}